2-dehydro-3-deoxy-D-gluconate 6-dehydrogenase activity [GO:0047000] (molecular function) Relationships: is a type of oxidoreductase activity, acting on the CH-OH group of donors, NAD or NADP as acceptor [GO:0016616] Definition: Catalysis of the reaction: 2-dehydro-3-deoxy-D-gluconate + NADP+ = (4S,5S)-4,5-dihydroxy-2,6-dioxohexanoate + H+ + NADPH. Sources: EC:1.1.1.126, RHEA:15109 Also known as: 2-dehydro-3-deoxy-D-gluconate:NADP+ 6-oxidoreductase activity, 2-keto-3-deoxy-D-gluconate dehydrogenase activity